positive regulation of zygospore formation [GO:0075299] (biological process) Relationships: is a type of positive regulation of sexual sporulation resulting in formation of a cellular spore [GO:0043941]; is a type of GO:0075298; positively regulates GO:0034296 Sources: GOC:pamgo_curators Definition: Any process that activates, maintains or increases the frequency, rate or extent of frequency, rate or extent of zygospore formation, a process in which a thick-walled spore of some algae and fungi is formed by union of two similar sexual cells, usually serves as a resting spore, and produces the sporophytic phase.